{
  "gene": "UniProtKB:P13284",
  "term_label": "oxidoreductase activity, acting on a sulfur group of donors",
  "gene_symbol": "IFI30",
  "gene_name": "Gamma-interferon-inducible lysosomal thiol reductase",
  "term_id": "GO:0016667"
}